cortisol metabolic process [GO:0034650] (biological process) Definition: The chemical reactions and pathways involving cortisol, the steroid hormone 11-beta-17,21-trihydroxypregn-4-ene-3,20-dione. Cortisol is synthesized from cholesterol in the adrenal gland and controls carbohydrate, fat and protein metabolism and has anti-inflammatory properties. Relationships: is a type of glucocorticoid metabolic process [GO:0008211]; is a type of GO:0034308; is a type of ketone metabolic process [GO:0042180]; is a type of GO:0120254; is_a GO:1902644 Also known as: cortisol metabolism Sources: GOC:BHF, GOC:mah, GOC:rl Subtypes: cortisol biosynthetic process [GO:0034651]